negative regulation of protein localization to basolateral plasma membrane [GO:1904509] (biological process) Definition: Any process that stops, prevents or reduces the frequency, rate or extent of protein localization to basolateral plasma membrane. Relationships: is a type of negative regulation of protein localization to cell periphery [GO:1904376]; is a type of regulation of protein localization to basolateral plasma membrane [GO:1904508]; is a type of negative regulation of protein localization to membrane [GO:1905476]; negatively regulates GO:1903361 Also known as: down regulation of protein localisation in basolateral plasma membrane, down regulation of protein localisation to basolateral plasma membrane, down regulation of protein localization in basolateral plasma membrane, down regulation of protein localization to basolateral plasma membrane, down-regulation of protein localisation in basolateral plasma membrane, down-regulation of protein localisation to basolateral plasma membrane, down-regulation of protein localization in basolateral plasma membrane, down-regulation of protein localization to basolateral plasma membrane, downregulation of protein localisation in basolateral plasma membrane, downregulation of protein localisation to basolateral plasma membrane, downregulation of protein localization in basolateral plasma membrane, downregulation of protein localization to basolateral plasma membrane, negative regulation of protein localisation in basolateral plasma membrane, negative regulation of protein localisation to basolateral plasma membrane, negative regulation of protein localization in basolateral plasma membrane, inhibition of protein localisation in basolateral plasma membrane, inhibition of protein localisation to basolateral plasma membrane, inhibition of protein localization in basolateral plasma membrane, inhibition of protein localization to basolateral plasma membrane References: PMID:26115433 Sources: GOC:TermGenie, GOC:kmv, GO_REF:0000058